{
  "term_label": "plasma membrane",
  "gene_name": "ADP-ribosylation factor-like protein 4C",
  "term_id": "GO:0005886",
  "gene": "UniProtKB:P56559",
  "gene_symbol": "ARL4C"
}